{
  "gene_symbol": "PEX7",
  "term_id": "GO:0016558",
  "gene_name": "Peroxisomal targeting signal 2 receptor",
  "gene": "UniProtKB:O00628",
  "term_label": "protein import into peroxisome matrix"
}